{
  "gene": "UniProtKB:Q86VX2",
  "term_id": "GO:0051059",
  "gene_symbol": "COMMD7",
  "gene_name": "COMM domain-containing protein 7",
  "term_label": "NF-kappaB binding"
}